{
  "term_id": "GO:0005737",
  "gene_symbol": "DAPK2",
  "gene": "UniProtKB:Q9UIK4",
  "term_label": "cytoplasm",
  "gene_name": "Death-associated protein kinase 2"
}